{
  "gene": "UniProtKB:Q7Z2F6",
  "gene_symbol": "KRBOX5",
  "gene_name": "KRAB domain-containing protein 5",
  "term_label": "nucleus",
  "term_id": "GO:0005634"
}